{
  "gene": "UniProtKB:Q5CZ79",
  "gene_name": "Ankyrin repeat domain-containing protein 20B",
  "term_id": "UNKNOWN:0003",
  "term_label": "Unknown cellular component",
  "gene_symbol": "ANKRD20A8P"
}